epithelial cell proliferation involved in renal tubule morphogenesis [GO:2001013] (biological process) Sources: GOC:obol Definition: Any epithelial cell proliferation that is involved in renal tubule morphogenesis. Subtypes: epithelial cell proliferation involved in Malpighian tubule morphogenesis [GO:0061331] Relationships: is a type of epithelial cell proliferation [GO:0050673]; is part of renal tubule morphogenesis [GO:0061333]